{
  "term_id": "UNKNOWN:0003",
  "term_label": "Unknown cellular component",
  "gene_symbol": "NUDT18",
  "gene": "UniProtKB:Q6ZVK8",
  "gene_name": "8-oxo-dGDP phosphatase NUDT18"
}